{
  "gene": "UniProtKB:Q9BR61",
  "gene_symbol": "ACBD6",
  "term_label": "fatty-acyl-CoA binding",
  "gene_name": "Acyl-CoA-binding domain-containing protein 6",
  "term_id": "GO:0000062"
}